regulation of auxin metabolic process [GO:0090354] (biological process) Subtypes: regulation of auxin biosynthetic process [GO:0010600], GO:0090355, negative regulation of auxin metabolic process [GO:0090356] Relationships: is a type of regulation of hormone metabolic process [GO:0032350]; regulates auxin metabolic process [GO:0009850] Sources: GOC:tb Also known as: regulation of auxin metabolism Definition: Any process that modulates the frequency, rate or extent of the chemical reactions and pathways involving auxins, plant hormones that regulate aspects of plant growth.